cap-dependent translation initiation factor activity [GO:0160296] (molecular function) Relationships: is a type of translation initiation factor activity [GO:0003743] Definition: A translation initiation factor activity that enables the recognition and binding to the 7-methylguanosine cap structure at the 5' end of eukaryotic mRNAs, promoting ribosome recruitment and assembly and translation initiation in a cap-dependent manner. References: PMID:31913484, PMID:32496897